oxidoreductase activity, acting on the CH-OH group of donors, quinone or similar compound as acceptor [GO:0016901] (molecular function) Definition: Catalysis of an oxidation-reduction (redox) reaction in which a CH-OH group acts as a hydrogen or electron donor and reduces a quinone or a similar acceptor molecule. Sources: EC:1.1.5.-, GOC:ai Relationships: is a type of GO:0016614 Subtypes: glycerol-3-phosphate dehydrogenase (quinone) activity [GO:0004368], quinoprotein glucose dehydrogenase activity [GO:0008876], GO:0008924, quinate dehydrogenase (quinone) activity [GO:0047519], fructose 5-dehydrogenase activity [GO:0047904], aldose sugar dehydrogenase activity [GO:0103040], GO:0140696, glucose dehydrogenase (FAD, quinone) activity [GO:0140762], GO:1990464